{
  "gene_symbol": "SLC25A17",
  "term_label": "AMP transmembrane transporter activity",
  "gene_name": "Peroxisomal membrane protein PMP34",
  "gene": "UniProtKB:O43808",
  "term_id": "GO:0080122"
}